{
  "term_id": "GO:0000922",
  "term_label": "spindle pole",
  "gene_symbol": "CENPF",
  "gene_name": "Centromere protein F",
  "gene": "UniProtKB:P49454"
}